{
  "term_label": "G protein-coupled glutamate receptor binding",
  "term_id": "GO:0035256",
  "gene_name": "Homer protein homolog 2",
  "gene_symbol": "HOMER2",
  "gene": "UniProtKB:Q9NSB8"
}